negative regulation of plasma lipoprotein oxidation [GO:0034445] (biological process) Definition: Any process that stops, prevents, or reduces the frequency, rate or extent of lipoprotein particle oxidation, occurring in the blood plasma. Sources: GOC:BHF, GOC:mah Also known as: inhibition of plasma lipoprotein oxidation, negative regulation of plasma lipoprotein particle oxidation Relationships: is a type of regulation of plasma lipoprotein oxidation [GO:0034444]; is a type of negative regulation of cellular component organization [GO:0051129]; is a type of GO:0051241; negatively regulates plasma lipoprotein particle oxidation [GO:0034441]